{
  "gene_name": "Protein FAM83C",
  "gene": "UniProtKB:Q9BQN1",
  "term_label": "protein kinase binding",
  "gene_symbol": "FAM83C",
  "term_id": "GO:0019901"
}